{
  "term_id": "GO:0019814",
  "gene_symbol": "IGLV1-44",
  "gene": "UniProtKB:P01699",
  "term_label": "immunoglobulin complex",
  "gene_name": "Immunoglobulin lambda variable 1-44"
}